{
  "term_label": "signaling adaptor activity",
  "gene_name": "TIR domain-containing adapter molecule 1",
  "term_id": "GO:0035591",
  "gene_symbol": "TICAM1",
  "gene": "UniProtKB:Q8IUC6"
}